{
  "term_label": "nucleoplasm",
  "gene_symbol": "RBM12",
  "term_id": "GO:0005654",
  "gene_name": "RNA-binding protein 12",
  "gene": "UniProtKB:Q9NTZ6"
}